{
  "gene": "UniProtKB:O60292",
  "term_label": "GTPase activator activity",
  "gene_name": "Signal-induced proliferation-associated 1-like protein 3",
  "gene_symbol": "SIPA1L3",
  "term_id": "GO:0005096"
}